{
  "gene": "UniProtKB:Q9Y4Z2",
  "term_id": "GO:0045944",
  "gene_name": "Neurogenin-3",
  "gene_symbol": "NEUROG3",
  "term_label": "positive regulation of transcription by RNA polymerase II"
}